carbon-nitrogen ligase activity, with glutamine as amido-N-donor [GO:0016884] (molecular function) Definition: Catalysis of the transfer of the amide nitrogen of glutamine to a substrate. Usually composed of two subunits or domains, one that first hydrolyzes glutamine, and then transfers the resulting ammonia to the second subunit (or domain), where it acts as a source of nitrogen. Relationships: is_a ligase activity, forming carbon-nitrogen bonds [GO:0016879] References: PMID:12360532 Subtypes: GO:0003922, NAD+ synthase (glutamine-hydrolyzing) activity [GO:0003952], asparagine synthase (glutamine-hydrolyzing) activity [GO:0004066], GO:0004088, GO:0004642, GO:0042242, hydrogenobyrinic acid a,c-diamide synthase (glutamine-hydrolysing) activity [GO:0043802], asparaginyl-tRNA synthase (glutamine-hydrolyzing) activity [GO:0050566], glutaminyl-tRNA synthase (glutamine-hydrolyzing) activity [GO:0050567], GO:0051921, GO:0140282